{
  "gene": "UniProtKB:P20810",
  "gene_symbol": "CAST",
  "term_id": "GO:0010859",
  "term_label": "calcium-dependent cysteine-type endopeptidase inhibitor activity",
  "gene_name": "Calpastatin"
}